{
  "gene_symbol": "TMEM88",
  "gene_name": "Transmembrane protein 88",
  "term_label": "plasma membrane",
  "gene": "UniProtKB:Q6PEY1",
  "term_id": "GO:0005886"
}